9+2 non-motile cilium [GO:0097732] (cellular component) Definition: A non-motile cilium where the axoneme has a ring of nine outer microtubule doublets plus two central microtubules (and is therefore called a 9+2 axoneme). References: PMID:21307074, PMID:22118931 Sources: GOC:cilia Also known as: non-motile 9+2 cilium, 9+2 immotile cilium Subtypes: kinocilium [GO:0060091] Relationships: is a type of non-motile cilium [GO:0097730]; has part outer dynein arm [GO:0036157] Note: This type of cilia may be present in solitary (e.g. in inner hair cells) or in multiple copies (e.g. in olfactory neurons).